endosome to plasma membrane protein transport [GO:0099638] (biological process) Subtypes: neurotransmitter receptor transport, endosome to plasma membrane [GO:0099639] Regulation: regulated by regulation of endosome to plasma membrane protein transport [GO:1905749]; negatively regulated by negative regulation of endosome to plasma membrane protein transport [GO:1905750]; positively regulated by positive regulation of endosome to plasma membrane protein transport [GO:1905751] Relationships: is a type of intracellular protein transport [GO:0006886]; is a type of endocytic recycling [GO:0032456]; is a type of establishment of protein localization to plasma membrane [GO:0061951]; is a type of protein localization to plasma membrane [GO:0072659] Sources: GOC:dos Definition: The directed movement of proteins from the endosome to the plasma membrane in transport vesicles.